{
  "term_label": "lateral element",
  "term_id": "GO:0000800",
  "gene_name": "Meiosis-specific protein MEI4",
  "gene": "UniProtKB:A8MW99",
  "gene_symbol": "MEI4"
}